{
  "term_label": "cytosol",
  "gene_name": "Gastrotropin",
  "term_id": "GO:0005829",
  "gene_symbol": "FABP6",
  "gene": "UniProtKB:P51161"
}